{
  "term_label": "Unknown cellular component",
  "gene_name": "Phosphatase and actin regulator 4",
  "term_id": "UNKNOWN:0003",
  "gene": "UniProtKB:Q8IZ21",
  "gene_symbol": "PHACTR4"
}